{
  "gene": "UniProtKB:O60462",
  "gene_symbol": "NRP2",
  "gene_name": "Neuropilin-2",
  "term_id": "GO:0017154",
  "term_label": "semaphorin receptor activity"
}